regulation of lipid catabolic process [GO:0050994] (biological process) Definition: Any process that modulates the frequency, rate, or extent of the chemical reactions and pathways resulting in the breakdown of lipids. Sources: GOC:ai Also known as: regulation of lipid breakdown, regulation of lipid catabolism, regulation of lipid degradation Relationships: is a type of regulation of catabolic process [GO:0009894]; is a type of GO:0019216; regulates GO:0016042 Subtypes: regulation of triglyceride catabolic process [GO:0010896], regulation of glucocorticoid catabolic process [GO:0031949], regulation of fatty acid beta-oxidation [GO:0031998], GO:0045952, negative regulation of lipid catabolic process [GO:0050995], positive regulation of lipid catabolic process [GO:0050996], regulation of phospholipid catabolic process [GO:0060696], regulation of palmitic acid catabolic process [GO:0106393], regulation of butyryl-CoA catabolic process to butanol [GO:1900497], regulation of butyryl-CoA catabolic process to butyrate [GO:1900500], regulation of prostaglandin catabolic process [GO:1905828], regulation of glucosylceramide catabolic process [GO:2000752]